{
  "term_id": "UNKNOWN:0003",
  "gene": "UniProtKB:A0A2R8YED5",
  "gene_name": "Olfactory receptor",
  "term_label": "Unknown cellular component",
  "gene_symbol": "OR5BS1"
}